positive regulation of trophectodermal cell proliferation [GO:1904075] (biological process) Definition: Any process that activates or increases the frequency, rate or extent of trophectodermal cell proliferation. References: PMID:24508636 Sources: GOC:TermGenie, GO_REF:0000058 Also known as: positive regulation of trophectoderm cell proliferation, up regulation of trophectoderm cell proliferation, up regulation of trophectodermal cell proliferation, up-regulation of trophectoderm cell proliferation, up-regulation of trophectodermal cell proliferation, upregulation of trophectoderm cell proliferation, upregulation of trophectodermal cell proliferation, activation of trophectoderm cell proliferation, activation of trophectodermal cell proliferation Relationships: is a type of positive regulation of cell population proliferation [GO:0008284]; is a type of regulation of trophectodermal cell proliferation [GO:1904073]; RO_0002213 GO:0001834